{
  "gene": "UniProtKB:Q969J2",
  "term_id": "GO:0006357",
  "gene_symbol": "ZKSCAN4",
  "term_label": "regulation of transcription by RNA polymerase II",
  "gene_name": "Zinc finger protein with KRAB and SCAN domains 4"
}